cardiac muscle tissue growth [GO:0055017] (biological process) Subtypes: cardiac muscle tissue growth involved in heart morphogenesis [GO:0003245] Also known as: heart muscle growth Relationships: is a type of developmental growth [GO:0048589]; is part of cardiac muscle tissue development [GO:0048738]; is part of heart growth [GO:0060419] Sources: GOC:devbiol Definition: The increase in size or mass of a cardiac muscle, where the increase in size or mass has the specific outcome of the progression of the organism over time from one condition to another. Regulation: regulated by regulation of cardiac muscle tissue growth [GO:0055021]; negatively regulated by negative regulation of cardiac muscle tissue growth [GO:0055022]; positively regulated by GO:0055023